{
  "gene_name": "Zinc finger and SCAN domain-containing protein 5B",
  "term_label": "regulation of transcription by RNA polymerase II",
  "gene": "UniProtKB:A6NJL1",
  "gene_symbol": "ZSCAN5B",
  "term_id": "GO:0006357"
}